{
  "gene": "UniProtKB:P15976",
  "gene_name": "Erythroid transcription factor",
  "gene_symbol": "GATA1",
  "term_id": "GO:0000981",
  "term_label": "DNA-binding transcription factor activity, RNA polymerase II-specific"
}